{
  "gene": "UniProtKB:O95180",
  "term_label": "high voltage-gated calcium channel activity",
  "term_id": "GO:0008331",
  "gene_name": "Voltage-dependent T-type calcium channel subunit alpha-1H",
  "gene_symbol": "CACNA1H"
}